{
  "term_id": "UNKNOWN:0002",
  "term_label": "Unknown biological process",
  "gene": "UniProtKB:Q7Z392",
  "gene_symbol": "TRAPPC11",
  "gene_name": "Trafficking protein particle complex subunit 11"
}